Lsm2-8 complex [GO:0120115] (cellular component) References: PMID:19121818, PMID:23221597, PMID:27627834, PMID:28768202 Sources: GOC:bhm, GOC:krc Relationships: is a type of Sm-like protein family complex [GO:0120114] Definition: A heteroheptameric, nuclear protein complex composed of Lsm2, Lsm3, Lsm4, Lsm5, Lsm6, Lsm7, and Lsm8, or orthologs thereof, that selectively binds to snRNAs, in particular U6 or U6atac snRNAs, and also to unspliced transcripts localized within the nucleus.